{
  "term_label": "O-fucosylpeptide 3-beta-N-acetylglucosaminyltransferase activity",
  "gene": "UniProtKB:Q9Y644",
  "term_id": "GO:0033829",
  "gene_name": "Beta-1,3-N-acetylglucosaminyltransferase radical fringe",
  "gene_symbol": "RFNG"
}